{
  "term_id": "GO:0005737",
  "term_label": "cytoplasm",
  "gene_name": "Rho guanine nucleotide exchange factor 6",
  "gene_symbol": "ARHGEF6",
  "gene": "UniProtKB:Q15052"
}